{
  "term_id": "GO:0051382",
  "term_label": "kinetochore assembly",
  "gene": "UniProtKB:P0DPK5",
  "gene_symbol": "H3Y2",
  "gene_name": "Histone H3.X"
}